{
  "gene_name": "Charged multivesicular body protein 3",
  "gene_symbol": "CHMP3",
  "term_label": "ESCRT III complex",
  "gene": "UniProtKB:Q9Y3E7",
  "term_id": "GO:0000815"
}